{
  "gene_name": "Kinesin-like protein KIF18A",
  "term_label": "microtubule binding",
  "term_id": "GO:0008017",
  "gene_symbol": "KIF18A",
  "gene": "UniProtKB:Q8NI77"
}